{
  "gene_symbol": "WTIP",
  "gene_name": "Wilms tumor protein 1-interacting protein",
  "gene": "UniProtKB:A6NIX2",
  "term_label": "adherens junction",
  "term_id": "GO:0005912"
}